{
  "gene_symbol": "HLA-DRA",
  "term_id": "GO:0050870",
  "term_label": "positive regulation of T cell activation",
  "gene": "UniProtKB:P01903",
  "gene_name": "HLA class II histocompatibility antigen, DR alpha chain"
}